{
  "gene": "UniProtKB:Q14332",
  "term_label": "non-canonical Wnt signaling pathway",
  "gene_symbol": "FZD2",
  "term_id": "GO:0035567",
  "gene_name": "Frizzled-2"
}